{
  "gene_symbol": "TMUB1",
  "gene": "UniProtKB:Q9BVT8",
  "gene_name": "Transmembrane and ubiquitin-like domain-containing protein 1",
  "term_id": "UNKNOWN:0001",
  "term_label": "Unknown molecular function"
}